regulation of cell morphogenesis [GO:0022604] (biological process) Sources: GOC:isa_complete Also known as: negative regulation of cell shape and cell size, positive regulation of cell shape and cell size, regulation of cell shape and cell size Definition: Any process that modulates the frequency, rate or extent of cell morphogenesis. Cell morphogenesis is the developmental process in which the shape of a cell is generated and organized. Relationships: is a type of GO:0022603; RO_0002211 cell morphogenesis [GO:0000902] Subtypes: regulation of cell shape [GO:0008360], positive regulation of cell morphogenesis [GO:0010770], negative regulation of cell morphogenesis [GO:0010771], regulation of unidimensional cell growth [GO:0051510], GO:0061924, regulation of apical constriction involved in ventral furrow formation [GO:0110073], regulation of neuron projection arborization [GO:0150011], GO:1900447, regulation of dendrite extension [GO:1903859], regulation of platelet formation [GO:1905219], regulation of cell morphogenesis involved in conjugation with cellular fusion [GO:1905708], GO:2000039, regulation of lamellipodium morphogenesis [GO:2000392]